luteal cell differentiation [GO:1903728] (biological process) Definition: The process in which a relatively unspecialized cell acquires the specialized features of a luteal cell. Large luteal cells develop from granulosa cells. Small luteal cells develop from theca cells. Sources: GOC:TermGenie, GO_REF:0000086, MP:0001133 Relationships: is a type of cell differentiation [GO:0030154] Also known as: lutein cell differentiation